nitrile biosynthetic process [GO:0080028] (biological process) Subtypes: GO:0019756, GO:0097288, 3-cyano-L-alanine biosynthetic process [GO:1903560] Definition: The chemical reactions and pathways resulting in the formation of a nitrile, an organic compound containing trivalent nitrogen attached to one carbon atom. References: PMID:18987211 Relationships: is a type of GO:0009058; is a type of nitrile metabolic process [GO:0050898]